{
  "gene": "UniProtKB:Q16552",
  "gene_name": "Interleukin-17A",
  "term_id": "UNKNOWN:0003",
  "gene_symbol": "IL17A",
  "term_label": "Unknown cellular component"
}